{
  "gene_name": "Adhesion G protein-coupled receptor L1",
  "term_label": "axon",
  "term_id": "GO:0030424",
  "gene": "UniProtKB:O94910",
  "gene_symbol": "ADGRL1"
}